negative regulation of gene expression [GO:0010629] (biological process) Subtypes: GO:0001818, negative regulation of production of molecular mediator of immune response [GO:0002701], mRNA catabolic process [GO:0006402], transposable element silencing [GO:0010526], GO:0016441, negative regulation of translation [GO:0017148], regulatory ncRNA-mediated gene silencing [GO:0031047], programmed DNA elimination [GO:0031049], transcriptional attenuation [GO:0031555], GO:0033119, negative regulation of gene expression, epigenetic [GO:0045814], GO:0061157, GO:0140669, negative regulation of snoRNA processing [GO:1902797], negative regulation of protein maturation [GO:1903318], GO:1903799, negative regulation of rRNA processing [GO:2000233], negative regulation of tRNA processing [GO:2000236] Note: This term covers any process that negatively regulates the rate of production of a mature gene product, and so includes processes that negatively regulate that rate by reducing the level, stability or availability of intermediates in the process of gene expression. For example, it covers any process that reduces the level, stability or availability of mRNA or circRNA for translation and thereby reduces the rate of production of the encoded protein via translation. Relationships: is a type of regulation of gene expression [GO:0010468]; is a type of negative regulation of macromolecule biosynthetic process [GO:0010558]; negatively regulates gene expression [GO:0010467] Definition: Any process that decreases the frequency, rate or extent of gene expression. Gene expression is the process in which a gene's coding sequence is converted into a mature gene product (protein or RNA). Sources: GOC:txnOH-2018 Also known as: gene silencing